{
  "gene_symbol": "TMOD4",
  "gene": "UniProtKB:Q9NZQ9",
  "term_id": "GO:0005865",
  "term_label": "striated muscle thin filament",
  "gene_name": "Tropomodulin-4"
}